{
  "gene": "UniProtKB:Q86SG4",
  "term_id": "GO:0005634",
  "gene_name": "Putative Dresden prostate carcinoma protein 2",
  "term_label": "nucleus",
  "gene_symbol": "HMGN2P46"
}